{
  "gene": "UniProtKB:Q9Y227",
  "gene_name": "Ectonucleoside triphosphate diphosphohydrolase 4",
  "term_label": "ribonucleoside triphosphate phosphatase activity",
  "gene_symbol": "ENTPD4",
  "term_id": "GO:0017111"
}